{
  "gene_name": "Cytosol aminopeptidase",
  "gene_symbol": "LAP3",
  "term_label": "cytoplasm",
  "term_id": "GO:0005737",
  "gene": "UniProtKB:P28838"
}